dihydropteroate synthase activity [GO:0004156] (molecular function) Sources: EC:2.5.1.15 Relationships: is a type of transferase activity, transferring alkyl or aryl (other than methyl) groups [GO:0016765] Also known as: (2-amino-4-hydroxy-7,8-dihydropteridin-6-yl)methyl-diphosphate:4-aminobenzoate 2-amino-4-hydroxydihydropteridine-6-methenyltransferase activity, 2-amino-4-hydroxy-6-hydroxymethyl-7,8-dihydropteridine-diphosphate:4-aminobenzoate 2-amino-4-hydroxydihydropteridine-6-methenyltransferase activity, 7,8-dihydropteroate synthase activity, 7,8-dihydropteroate synthetase activity, 7,8-dihydropteroic acid synthetase activity, DHPS activity, dihydropteroate diphosphorylase activity, dihydropteroate pyrophosphorylase activity, dihydropteroate synthetase activity, dihydropteroic synthetase activity Definition: Catalysis of the reaction: 2-amino-4-hydroxy-6-hydroxymethyl-7,8-dihydropteridine diphosphate + 4-aminobenzoate = diphosphate + dihydropteroate.